{
  "gene_name": "Transmembrane and immunoglobulin domain-containing protein 1",
  "gene_symbol": "TMIGD1",
  "term_label": "Unknown biological process",
  "gene": "UniProtKB:Q6UXZ0",
  "term_id": "UNKNOWN:0002"
}